{
  "term_label": "asparagine synthase (glutamine-hydrolyzing) activity",
  "gene": "UniProtKB:P08243",
  "term_id": "GO:0004066",
  "gene_name": "Asparagine synthetase [glutamine-hydrolyzing]",
  "gene_symbol": "ASNS"
}